{
  "gene_symbol": "APOBEC3D",
  "term_id": "GO:0000932",
  "term_label": "P-body",
  "gene": "UniProtKB:Q96AK3",
  "gene_name": "DNA dC-dU-editing enzyme APOBEC-3D"
}